regulation of sphingomyelin catabolic process [GO:2000754] (biological process) Also known as: regulation of sphingomyelin breakdown, regulation of sphingomyelin catabolism, regulation of sphingomyelin degradation Relationships: is a type of regulation of amide metabolic process [GO:0034248]; is a type of regulation of phospholipid catabolic process [GO:0060696]; is a type of GO:1905038; regulates GO:0006685 Definition: Any process that modulates the frequency, rate or extent of sphingomyelin catabolic process. Sources: GOC:BHF Subtypes: positive regulation of sphingomyelin catabolic process [GO:2000755]